granulosa cell development [GO:0060016] (biological process) Definition: The process whose specific outcome is the progression of a granulosa cell over time, from its formation to the mature structure. Cell development does not include the steps involved in committing a cell to a granulosa cell fate. Sources: GOC:dph Relationships: is a type of epithelial cell development [GO:0002064]; is part of granulosa cell differentiation [GO:0060014]